{
  "term_label": "olfactory receptor activity",
  "term_id": "GO:0004984",
  "gene": "UniProtKB:Q8NGG3",
  "gene_symbol": "OR5T3",
  "gene_name": "Olfactory receptor 5T3"
}